{
  "gene": "UniProtKB:Q8NCH0",
  "gene_symbol": "CHST14",
  "term_id": "UNKNOWN:0003",
  "term_label": "Unknown cellular component",
  "gene_name": "Carbohydrate sulfotransferase 14"
}